{
  "term_label": "polyubiquitin modification-dependent protein binding",
  "term_id": "GO:0031593",
  "gene_symbol": "AFG2B",
  "gene_name": "ATPase family gene 2 protein homolog B",
  "gene": "UniProtKB:Q9BVQ7"
}